negative regulation of myeloid dendritic cell activation [GO:0030886] (biological process) Sources: GOC:mah Also known as: down regulation of myeloid dendritic cell activation, down-regulation of myeloid dendritic cell activation, downregulation of myeloid dendritic cell activation, inhibition of myeloid dendritic cell activation Relationships: is a type of negative regulation of leukocyte activation [GO:0002695]; is a type of regulation of myeloid dendritic cell activation [GO:0030885]; negatively regulates myeloid dendritic cell activation [GO:0001773] Definition: Any process that stops, prevents, or reduces the frequency, rate or extent of myeloid dendritic cell activation.